{
  "term_id": "GO:0036064",
  "gene": "UniProtKB:Q9BVV6",
  "gene_name": "Protein TALPID3",
  "term_label": "ciliary basal body",
  "gene_symbol": "KIAA0586"
}